{
  "gene_symbol": "ACSM2A",
  "gene_name": "Acyl-coenzyme A synthetase ACSM2A, mitochondrial",
  "term_id": "GO:0006637",
  "gene": "UniProtKB:Q08AH3",
  "term_label": "acyl-CoA metabolic process"
}